terpenoid catabolic process [GO:0016115] (biological process) Subtypes: GO:0016100, GO:0016103, GO:0016105, sesquiterpenoid catabolic process [GO:0016107], tetraterpenoid catabolic process [GO:0016110], polyterpenoid catabolic process [GO:0016113], farnesyl diphosphate catabolic process [GO:0045339], GO:1902247 Sources: GOC:ai Definition: The chemical reactions and pathways resulting in the breakdown of terpenoids, any member of a class of compounds characterized by an isoprenoid chemical structure. Relationships: is a type of terpenoid metabolic process [GO:0006721]; is a type of isoprenoid catabolic process [GO:0008300] Also known as: terpenoid breakdown, terpenoid catabolism, terpenoid degradation